{
  "term_id": "GO:0005829",
  "gene_symbol": "USP17L2",
  "gene_name": "Ubiquitin carboxyl-terminal hydrolase 17",
  "term_label": "cytosol",
  "gene": "UniProtKB:Q6R6M4"
}